{
  "term_label": "HCN channel complex",
  "gene_name": "Potassium_sodium hyperpolarization-activated cyclic nucleotide-gated channel 2",
  "gene_symbol": "HCN2",
  "term_id": "GO:0098855",
  "gene": "UniProtKB:Q9UL51"
}